apoptotic process involved in atrial ventricular junction remodeling [GO:0003296] (biological process) Also known as: apoptosis involved in atrial ventricular junction remodelling, apoptosis involved in atrio-ventricular junction remodeling, apoptosis involved in atrio-ventricular junction remodelling, apoptosis involved in atrioventricular junction remodeling, apoptosis involved in atrioventricular junction remodelling Sources: GOC:mtg_apoptosis, GOC:mtg_heart Definition: Any apoptotic process that contributes to the reorganization of tissue resulting in the maturation of the atrial ventricular junction. Relationships: is a type of GO:0003278; is part of atrial ventricular junction remodeling [GO:0003294]